histone H3K9 monomethyltransferase activity [GO:0140948] (molecular function) Sources: RHEA:60280 Note: Comment: Note that the residue position corresponds to the canonical human H3 histone (UniProtKB:P84243); this residue is conserved across all eukaryotes. Residue 1 is the first residue following removal of the initiating Methionine (Met). Note that each histone is encoded by multiple genes, and sequences may vary across different genes within an organism. Also known as: histone H3-K9 methylation, histone H3K9 methylation, histone H3K9 monomethylase activity, histone lysine N-monomethyltransferase activity (H3-K9 specific) Relationships: is a type of histone H3K9 methyltransferase activity [GO:0046974] Definition: Catalysis of the reaction: L-lysyl9-[histone H3] + S-adenosyl-L-methionine = H+ + N6-methyl-L-lysyl9-[histone H3] + S-adenosyl-L-homocysteine. This reaction is the addition of a methyl group to the unmethylated lysine residue at position 9 of histone H3, producing histone H3K9me.